positive regulation of parathyroid hormone secretion [GO:2000830] (biological process) Sources: GOC:obol Relationships: is a type of GO:0046887; is a type of GO:0051240; is a type of regulation of parathyroid hormone secretion [GO:2000828]; positively regulates GO:0035898 Also known as: positive regulation of PTH secretion, positive regulation of parathormone secretion, positive regulation of parathyrin secretion Definition: Any process that activates or increases the frequency, rate or extent of parathyroid hormone secretion.